polysaccharide localization [GO:0033037] (biological process) Definition: Any process in which a polysaccharide is transported to, or maintained in, a specific location. Also known as: polysaccharide localisation Subtypes: chitin localization [GO:0006033], callose localization [GO:0052545] Relationships: is_a GO:0033036 Sources: GOC:mah